{
  "gene_symbol": "BSX",
  "term_label": "DNA-binding transcription factor activity, RNA polymerase II-specific",
  "term_id": "GO:0000981",
  "gene_name": "Brain-specific homeobox protein homolog",
  "gene": "UniProtKB:Q3C1V8"
}